pyridine N-methyltransferase activity [GO:0030760] (molecular function) Relationships: is a type of S-adenosylmethionine-dependent methyltransferase activity [GO:0008757] Definition: Catalysis of the reaction: S-adenosyl-L-methionine(1+) + pyridine = N-methylpyridinium + S-adenosyl-L-homocysteine. Sources: EC:2.1.1.87, RHEA:16893 Also known as: S-adenosyl-L-methionine:pyridine N-methyltransferase activity, pyridine methyltransferase activity